{
  "term_id": "GO:0005874",
  "gene_name": "Dynamin-1",
  "term_label": "microtubule",
  "gene": "UniProtKB:Q05193",
  "gene_symbol": "DNM1"
}